{
  "gene_symbol": "SCT",
  "gene": "UniProtKB:P09683",
  "term_id": "GO:0005102",
  "term_label": "signaling receptor binding",
  "gene_name": "Secretin"
}